{
  "term_id": "GO:0005634",
  "term_label": "nucleus",
  "gene": "UniProtKB:Q8NC51",
  "gene_name": "SERPINE1 mRNA-binding protein 1",
  "gene_symbol": "SERBP1"
}